lateral mesodermal cell fate determination [GO:0048373] (biological process) Regulation: regulated by regulation of lateral mesodermal cell fate determination [GO:0048374]; negatively regulated by negative regulation of lateral mesodermal cell fate determination [GO:0048375]; positively regulated by GO:0048376 Definition: The process in which a cell becomes capable of differentiating autonomously into a lateral mesoderm cell regardless of its environment; upon determination, the cell fate cannot be reversed. Sources: GOC:jid Also known as: lateral mesoderm cell fate determination, lateral plate mesoderm cell fate determination, lateral plate mesodermal cell fate determination Relationships: is a type of mesodermal cell fate determination [GO:0007500]; is part of GO:0048372